negative regulation of peptidyl-lysine crotonylation [GO:0120094] (biological process) Definition: Any process that stops or reduces the rate of crotonylation of a lysine residue in a protein. References: PMID:28803779 Relationships: is a type of negative regulation of protein modification process [GO:0031400]; is a type of regulation of peptidyl-lysine crotonylation [GO:0120093]; negatively regulates peptidyl-lysine crotonylation [GO:0140066]